{
  "term_id": "GO:0046872",
  "gene_symbol": "MT2A",
  "gene_name": "Metallothionein-2",
  "gene": "UniProtKB:P02795",
  "term_label": "metal ion binding"
}